{
  "gene_name": "Vitamin K-dependent protein Z",
  "gene_symbol": "PROZ",
  "term_label": "extracellular space",
  "term_id": "GO:0005615",
  "gene": "UniProtKB:P22891"
}